microtubule bundle formation involved in horsetail-astral microtubule organization [GO:1903563] (biological process) Relationships: is a type of microtubule bundle formation [GO:0001578]; is a type of GO:1903046; BFO_0000050 horsetail-astral microtubule organization [GO:0032118] References: PMID:15647375 Sources: GOC:TermGenie, GO_REF:0000060 Definition: Any microtubule bundle formation that is involved in horsetail-astral microtubule organization. Also known as: microtubule bundle formation involved in horsetail-astral microtubule array organization, microtubule bundle formation involved in horsetail-astral microtubule organisation, microtubule bundling involved in horsetail-astral microtubule array organization, microtubule bundling involved in horsetail-astral microtubule organisation, microtubule bundling involved in horsetail-astral microtubule organization